{
  "term_id": "UNKNOWN:0003",
  "gene_name": "Ubiquitin carboxyl-terminal hydrolase 45",
  "gene": "UniProtKB:Q70EL2",
  "gene_symbol": "USP45",
  "term_label": "Unknown cellular component"
}